{
  "gene": "UniProtKB:Q86W47",
  "gene_name": "Calcium-activated potassium channel subunit beta-4",
  "term_id": "GO:0015459",
  "gene_symbol": "KCNMB4",
  "term_label": "potassium channel regulator activity"
}